positive regulation of meiotic DNA double-strand break formation involved in reciprocal meiotic recombination [GO:1905263] (biological process) Relationships: is a type of positive regulation of meiotic DNA double-strand break formation [GO:1903343]; is_a GO:1905261; positively regulates GO:0010780 References: PMID:26653857 Sources: GOC:TermGenie, GO_REF:0000058 Also known as: up regulation of meiotic DNA double-strand break formation involved in reciprocal meiotic recombination, up-regulation of meiotic DNA double-strand break formation involved in reciprocal meiotic recombination, upregulation of meiotic DNA double-strand break formation involved in reciprocal meiotic recombination, activation of meiotic DNA double-strand break formation involved in reciprocal meiotic recombination Definition: Any process that activates or increases the frequency, rate or extent of meiotic DNA double-strand break formation involved in reciprocal meiotic recombination.